{
  "term_label": "nucleus",
  "term_id": "GO:0005634",
  "gene": "UniProtKB:Q96DT7",
  "gene_name": "Zinc finger and BTB domain-containing protein 10",
  "gene_symbol": "ZBTB10"
}